{
  "gene_symbol": "RALGAPA1",
  "term_id": "GO:0005096",
  "term_label": "GTPase activator activity",
  "gene": "UniProtKB:Q6GYQ0",
  "gene_name": "Ral GTPase-activating protein subunit alpha-1"
}